{
  "term_label": "nucleus",
  "gene_symbol": "BEX4",
  "gene_name": "Protein BEX4",
  "term_id": "GO:0005634",
  "gene": "UniProtKB:Q9NWD9"
}